type II protein secretion system complex [GO:0015627] (cellular component) Definition: A large protein complex, containing 12-15 subunits, that spans the cell envelope of Gram-negative bacteria and mediates the movement of proteins into the extracellular environment. The complex includes a component in the cytoplasm, an inner membrane subcomplex that reaches into the periplasmic compartment and a secretion pore in the outer membrane. Proteins using the Type II pathway are transported across the cytoplasmic membrane by the Sec or Tat complex. References: PMID:16448494 Also known as: MTB, T2SS-associated complexes, main terminal branch, Sec-dependent secretion system-associated complex, general secretion pathway-associated complex Note: Note that the type II protein secretion system complex does not include components of the Sec or Tat pathways. For components of these pathways, consider annotating to 'cell envelope Sec complex ; GO:0031522' or 'TAT protein translocation system complex ; GO:0033281'. Relationships: is a type of protein-containing complex [GO:0032991]